maltose metabolic process [GO:0000023] (biological process) Relationships: is a type of GO:0005984 Also known as: malt sugar metabolic process, malt sugar metabolism, maltose metabolism Definition: The chemical reactions and pathways involving the disaccharide maltose (4-O-alpha-D-glucopyranosyl-D-glucopyranose), an intermediate in the catabolism of glycogen and starch. Subtypes: GO:0000024, maltose catabolic process [GO:0000025] Sources: GOC:jl, ISBN:0198506732